{
  "term_id": "GO:0007163",
  "gene": "UniProtKB:P60763",
  "gene_symbol": "RAC3",
  "gene_name": "Ras-related C3 botulinum toxin substrate 3",
  "term_label": "establishment or maintenance of cell polarity"
}